{
  "gene_name": "HCG1796489",
  "gene": "UniProtKB:A0A1B0GTJ6",
  "gene_symbol": "LOC101059948",
  "term_id": "UNKNOWN:0002",
  "term_label": "Unknown biological process"
}